MutSalpha complex [GO:0032301] (cellular component) Definition: A heterodimer involved in the recognition and repair of base-base and small insertion/deletion mismatches. In human the complex consists of two subunits, MSH2 and MSH6. References: PMID:11005803 Also known as: MMR complex, MSH2/MSH6 complex Relationships: is a type of mismatch repair complex [GO:0032300]; is a type of nuclear protein-containing complex [GO:0140513]